carbohydrate transmembrane transport [GO:0034219] (biological process) Sources: GOC:mah Definition: The process in which a carbohydrate is transported across a membrane. Relationships: is a type of carbohydrate transport [GO:0008643]; is a type of GO:0055085 Note: Note that this term is not intended for use in annotating lateral movement within membranes. Subtypes: L-idonate transmembrane transport [GO:0015726], monosaccharide transmembrane transport [GO:0015749], GO:0015778, arabinitol transmembrane transport [GO:0015792], GO:0015793, GO:0015795, GO:0015796, mannitol transmembrane transport [GO:0015797], D-glucarate transmembrane transport [GO:0042870], D-galactonate transmembrane transport [GO:0042875], GO:0042899, glucosylglycerol transmembrane transport [GO:0051475], carbohydrate import across plasma membrane [GO:0098704], GO:1901975, xylitol transmembrane transport [GO:1902341], maltose transmembrane transport [GO:1904981], GO:1904982 Also known as: carbohydrate membrane transport, transmembrane carbohydrate transport